{
  "term_label": "Golgi membrane",
  "gene_symbol": "B3GALNT2",
  "gene_name": "UDP-GalNAc:beta-1,3-N-acetylgalactosaminyltransferase 2",
  "term_id": "GO:0000139",
  "gene": "UniProtKB:Q8NCR0"
}